{
  "term_label": "Unknown biological process",
  "gene": "UniProtKB:Q567V2",
  "gene_name": "Mpv17-like protein 2",
  "gene_symbol": "MPV17L2",
  "term_id": "UNKNOWN:0002"
}